alpha3-beta1 integrin-thrombospondin complex [GO:0071095] (cellular component) References: PMID:11358957 Also known as: ITGA3-ITGB1-THBS1 complex Definition: A protein complex that consists of an alpha3-beta1 integrin complex bound to thrombospondin. Relationships: is a type of plasma membrane protein complex [GO:0098797]